{
  "term_id": "GO:0005634",
  "gene_name": "Paired mesoderm homeobox protein 2",
  "gene": "UniProtKB:Q99811",
  "term_label": "nucleus",
  "gene_symbol": "PRRX2"
}